{
  "term_label": "cell adhesion molecule binding",
  "gene": "UniProtKB:O95206",
  "gene_symbol": "PCDH8",
  "term_id": "GO:0050839",
  "gene_name": "Protocadherin-8"
}